{
  "gene": "UniProtKB:Q9Y2U9",
  "term_id": "UNKNOWN:0003",
  "gene_name": "Kelch domain-containing protein 2",
  "term_label": "Unknown cellular component",
  "gene_symbol": "KLHDC2"
}